{
  "gene_symbol": "OR13C3",
  "gene": "UniProtKB:Q8NGS6",
  "term_label": "detection of chemical stimulus involved in sensory perception of smell",
  "term_id": "GO:0050911",
  "gene_name": "Olfactory receptor 13C3"
}